positive regulation of helicase activity [GO:0051096] (biological process) Sources: GOC:ai Relationships: is a type of positive regulation of ATP-dependent activity [GO:0032781]; is_a positive regulation of catalytic activity [GO:0043085]; positively regulates helicase activity [GO:0004386] Also known as: up regulation of helicase activity, up-regulation of helicase activity, upregulation of helicase activity, activation of helicase activity, stimulation of helicase activity Definition: Any process that activates or increases the activity of a helicase.